{
  "gene_symbol": "ACOX2",
  "term_label": "peroxisome",
  "gene_name": "Peroxisomal acyl-coenzyme A oxidase 2",
  "term_id": "GO:0005777",
  "gene": "UniProtKB:Q99424"
}